{
  "gene": "UniProtKB:Q6RVD6",
  "term_label": "Unknown molecular function",
  "term_id": "UNKNOWN:0001",
  "gene_name": "Spermatogenesis-associated protein 8",
  "gene_symbol": "SPATA8"
}